{
  "gene_name": "Small integral membrane protein 19",
  "gene_symbol": "SMIM19",
  "term_label": "Unknown cellular component",
  "gene": "UniProtKB:Q96E16",
  "term_id": "UNKNOWN:0003"
}